{
  "term_id": "GO:0005634",
  "term_label": "nucleus",
  "gene_symbol": "ZNF81",
  "gene": "UniProtKB:P51508",
  "gene_name": "Zinc finger protein 81"
}